{
  "term_label": "Unknown molecular function",
  "term_id": "UNKNOWN:0001",
  "gene": "UniProtKB:Q9Y2S7",
  "gene_name": "Polymerase delta-interacting protein 2",
  "gene_symbol": "POLDIP2"
}